chemorepulsion of dopaminergic neuron axon [GO:0036518] (biological process) Also known as: chemorepulsion of DA axon, chemorepulsion of dopaminergic axon Definition: The process in which a dopaminergic neuron growth cone is directed to a specific target site in response to a repulsive chemical cue. References: PMID:21106844, PMID:23517308 Sources: GOC:PARL, GOC:bf Relationships: is a type of chemorepulsion of axon [GO:0061643]; is part of dopaminergic neuron axon guidance [GO:0036514]